{
  "term_id": "GO:2000042",
  "gene_name": "DNA helicase B",
  "gene": "UniProtKB:Q8NG08",
  "term_label": "negative regulation of double-strand break repair via homologous recombination",
  "gene_symbol": "HELB"
}